{
  "term_id": "GO:2001224",
  "gene_name": "NMDA receptor synaptonuclear signaling and neuronal migration factor",
  "term_label": "positive regulation of neuron migration",
  "gene": "UniProtKB:Q6X4W1",
  "gene_symbol": "NSMF"
}